{
  "gene": "UniProtKB:Q02575",
  "gene_name": "Helix-loop-helix protein 1",
  "term_id": "UNKNOWN:0003",
  "term_label": "Unknown cellular component",
  "gene_symbol": "NHLH1"
}